{
  "gene_name": "Tubulin polyglutamylase TTLL11",
  "term_label": "microtubule cytoskeleton organization",
  "gene": "UniProtKB:Q8NHH1",
  "term_id": "GO:0000226",
  "gene_symbol": "TTLL11"
}